{
  "gene_symbol": "CREBBP",
  "term_label": "transcription regulator complex",
  "gene": "UniProtKB:Q92793",
  "term_id": "GO:0005667",
  "gene_name": "CREB-binding protein"
}